{
  "term_id": "GO:0000981",
  "gene_symbol": "SP1",
  "term_label": "DNA-binding transcription factor activity, RNA polymerase II-specific",
  "gene": "UniProtKB:P08047",
  "gene_name": "Transcription factor Sp1"
}